{
  "gene": "UniProtKB:O00400",
  "gene_name": "Acetyl-coenzyme A transporter 1",
  "gene_symbol": "SLC33A1",
  "term_label": "acetyl-CoA transmembrane transporter activity",
  "term_id": "GO:0008521"
}